{
  "term_id": "GO:0031856",
  "gene_symbol": "PTH",
  "gene": "UniProtKB:P01270",
  "gene_name": "Parathyroid hormone",
  "term_label": "parathyroid hormone receptor binding"
}